{
  "term_label": "very-low-density lipoprotein particle",
  "gene": "UniProtKB:Q6Q788",
  "term_id": "GO:0034361",
  "gene_symbol": "APOA5",
  "gene_name": "Apolipoprotein A-V"
}